{
  "gene_name": "1-phosphatidylinositol 4,5-bisphosphate phosphodiesterase gamma-1",
  "gene": "UniProtKB:P19174",
  "term_id": "GO:0004435",
  "gene_symbol": "PLCG1",
  "term_label": "phosphatidylinositol-4,5-bisphosphate phospholipase C activity"
}